{
  "gene_name": "Cornifin-B",
  "term_id": "UNKNOWN:0002",
  "term_label": "Unknown biological process",
  "gene_symbol": "SPRR1B",
  "gene": "UniProtKB:P22528"
}